{
  "gene_symbol": "TMEM50A",
  "gene": "UniProtKB:O95807",
  "term_id": "UNKNOWN:0003",
  "term_label": "Unknown cellular component",
  "gene_name": "Transmembrane protein 50A"
}